{
  "gene_name": "Homocysteine-responsive endoplasmic reticulum-resident ubiquitin-like domain member 1 protein",
  "term_label": "transmembrane transporter binding",
  "term_id": "GO:0044325",
  "gene": "UniProtKB:Q15011",
  "gene_symbol": "HERPUD1"
}